{
  "term_label": "R-SMAD binding",
  "gene_name": "Protein TMEPAI",
  "gene_symbol": "PMEPA1",
  "gene": "UniProtKB:Q969W9",
  "term_id": "GO:0070412"
}